{
  "term_id": "GO:0003682",
  "term_label": "chromatin binding",
  "gene_name": "E3 ubiquitin-protein ligase RING2",
  "gene": "UniProtKB:Q99496",
  "gene_symbol": "RNF2"
}